{
  "gene": "UniProtKB:P0DSO1",
  "gene_name": "Protein FAM246C",
  "term_label": "Unknown molecular function",
  "gene_symbol": "FAM246C",
  "term_id": "UNKNOWN:0001"
}